{
  "gene_name": "Pinin",
  "gene": "UniProtKB:Q9H307",
  "gene_symbol": "PNN",
  "term_label": "catalytic step 2 spliceosome",
  "term_id": "GO:0071013"
}